{
  "gene_name": "Putative cytochrome P450 2D7",
  "term_id": "GO:0005737",
  "gene_symbol": "CYP2D7",
  "term_label": "cytoplasm",
  "gene": "UniProtKB:A0A087X1C5"
}